{
  "term_id": "GO:0005615",
  "gene_symbol": "CSH2",
  "term_label": "extracellular space",
  "gene_name": "Chorionic somatomammotropin hormone 2",
  "gene": "UniProtKB:P0DML3"
}